3-isopropylmalate dehydratase complex [GO:0009316] (cellular component) Also known as: isopropylmalate isomerase complex Note: See also the molecular function term '3-isopropylmalate dehydratase activity ; GO:0003861'. References: PMID:7026530 Sources: GOC:jl, MetaCyc:3-ISOPROPYLMALISOM-CPLX Definition: A heterodimeric enzyme complex composed of subunits leuC and leuD. Catalyzes the isomerization between 2-isopropylmalate and 3-isopropylmalate, via the formation of 2-isopropylmaleate. Relationships: is a type of catalytic complex [GO:1902494]; is part of cytosol [GO:0005829]